{
  "gene_symbol": "ATXN7L3B",
  "gene_name": "Ataxin-7-like protein 3B",
  "term_label": "regulation of gene expression",
  "gene": "UniProtKB:Q96GX2",
  "term_id": "GO:0010468"
}